{
  "gene_name": "Inactive Rho GTPase-activating protein 11B",
  "gene_symbol": "ARHGAP11B",
  "term_id": "UNKNOWN:0002",
  "gene": "UniProtKB:Q3KRB8",
  "term_label": "Unknown biological process"
}